{
  "term_id": "GO:0000978",
  "gene_name": "Transcription factor 12",
  "gene_symbol": "TCF12",
  "term_label": "RNA polymerase II cis-regulatory region sequence-specific DNA binding",
  "gene": "UniProtKB:Q99081"
}